{
  "term_id": "UNKNOWN:0001",
  "gene_name": "Proteasome assembly chaperone 4",
  "gene": "UniProtKB:Q5JS54",
  "term_label": "Unknown molecular function",
  "gene_symbol": "PSMG4"
}